{
  "gene": "UniProtKB:Q68DY9",
  "term_id": "GO:0000978",
  "gene_name": "Zinc finger protein 772",
  "gene_symbol": "ZNF772",
  "term_label": "RNA polymerase II cis-regulatory region sequence-specific DNA binding"
}